{
  "gene_symbol": "ESRG",
  "term_id": "UNKNOWN:0003",
  "gene_name": "Embryonic stem cell-related gene protein",
  "gene": "UniProtKB:Q1W209",
  "term_label": "Unknown cellular component"
}